{
  "gene": "UniProtKB:O75607",
  "term_label": "RNA binding",
  "term_id": "GO:0003723",
  "gene_symbol": "NPM3",
  "gene_name": "Nucleoplasmin-3"
}